{
  "term_label": "cytoplasmic microtubule organization",
  "gene": "UniProtKB:Q9UGJ1",
  "gene_name": "Gamma-tubulin complex component 4",
  "term_id": "GO:0031122",
  "gene_symbol": "TUBGCP4"
}